{
  "term_id": "GO:0010385",
  "gene_symbol": "ZNF445",
  "term_label": "double-stranded methylated DNA binding",
  "gene": "UniProtKB:P59923",
  "gene_name": "Zinc finger protein 445"
}